{
  "gene": "UniProtKB:Q9NPA8",
  "term_label": "transcription coactivator activity",
  "gene_symbol": "ENY2",
  "term_id": "GO:0003713",
  "gene_name": "Transcription and mRNA export factor ENY2"
}